mitotic spindle polar microtubule [GO:1990537] (CC) Relationships: is a type of GO:0005827; is a type of mitotic spindle microtubule [GO:1990498] References: PMID:16079915 Definition: Any of the mitotic spindle microtubules that come from each pole and overlap at the spindle midzone.